{
  "gene": "UniProtKB:Q8N3H0",
  "gene_name": "Chemokine-like protein TAFA-2",
  "term_id": "GO:0005615",
  "gene_symbol": "TAFA2",
  "term_label": "extracellular space"
}